{
  "gene_symbol": "GUCY1B1",
  "term_label": "guanylate cyclase activity",
  "term_id": "GO:0004383",
  "gene_name": "Guanylate cyclase soluble subunit beta-1",
  "gene": "UniProtKB:Q02153"
}